{
  "term_id": "UNKNOWN:0003",
  "gene_symbol": "PTF1A",
  "gene_name": "Pancreas transcription factor 1 subunit alpha",
  "term_label": "Unknown cellular component",
  "gene": "UniProtKB:Q7RTS3"
}